protein-RNA covalent cross-linking repair [GO:0160127] (biological process) Relationships: is a type of rescue of stalled ribosome [GO:0072344] Definition: A process that rescues stalled ribosomes by removing the covalent cross-link between RNA and a protein. References: PMID:37951215, PMID:37951216